{
  "term_label": "Unknown molecular function",
  "gene_symbol": "LINC00518",
  "gene": "UniProtKB:Q8N0U6",
  "term_id": "UNKNOWN:0001",
  "gene_name": "Putative uncharacterized protein encoded by LINC00518"
}